{
  "gene_symbol": "PPIL6",
  "gene": "UniProtKB:Q8IXY8",
  "term_id": "GO:0005737",
  "term_label": "cytoplasm",
  "gene_name": "Probable inactive peptidyl-prolyl cis-trans isomerase-like 6"
}